{
  "term_label": "Unknown molecular function",
  "gene_name": "Splicing regulatory glutamine_lysine-rich protein 1",
  "gene_symbol": "SREK1",
  "gene": "UniProtKB:Q8WXA9",
  "term_id": "UNKNOWN:0001"
}